{
  "term_id": "GO:0007264",
  "gene": "UniProtKB:Q96HU8",
  "gene_name": "GTP-binding protein Di-Ras2",
  "gene_symbol": "DIRAS2",
  "term_label": "small GTPase-mediated signal transduction"
}